proteasome-nuclear membrane anchor activity [GO:1990919] (molecular function) Relationships: is_a protein-membrane adaptor activity [GO:0043495] Definition: The binding activity of a molecule that brings together a proteasome complex and a nuclear inner membrane, to maintain the nuclear membrane localization of the proteasome. References: PMID:16096059 Also known as: nuclear membrane proteasome anchor, nuclear membrane proteasome tether, nuclear membrane proteasome tether activity, nuclear membrane-proteasome anchor activity, nuclear membrane-proteasome tether activity, nuclear membrane proteasome adaptor, tethering factor for nuclear proteasome